adenosine receptor binding [GO:0031685] (molecular function) Also known as: adenosine receptor ligand Sources: GOC:mah, GOC:nln Definition: Binding to an adenosine receptor. Relationships: is a type of G protein-coupled receptor binding [GO:0001664] Subtypes: A1 adenosine receptor binding [GO:0031686], A2A adenosine receptor binding [GO:0031687], A2B adenosine receptor binding [GO:0031688], A3 adenosine receptor binding [GO:0031689]